{
  "gene": "UniProtKB:Q8IXQ5",
  "gene_name": "Kelch-like protein 7",
  "term_id": "GO:0005737",
  "gene_symbol": "KLHL7",
  "term_label": "cytoplasm"
}